{
  "gene": "UniProtKB:Q92913",
  "term_label": "neurogenesis",
  "gene_name": "Fibroblast growth factor 13",
  "term_id": "GO:0022008",
  "gene_symbol": "FGF13"
}